{
  "gene_name": "Double-stranded RNA-binding protein Staufen homolog 2",
  "gene": "UniProtKB:Q9NUL3",
  "gene_symbol": "STAU2",
  "term_label": "neuron projection",
  "term_id": "GO:0043005"
}